L-leucine transport [GO:0015820] (biological process) Sources: GOC:ai Definition: The directed movement of L-leucine, 2-amino-4-methylpentanoic acid, into, out of or within a cell, or between cells, by means of some agent such as a transporter or pore. Subtypes: GO:1903801 Also known as: leucine transport Relationships: is a type of organic cation transport [GO:0015695]; is a type of branched-chain amino acid transport [GO:0015803]; is a type of neutral amino acid transport [GO:0015804]; is a type of L-amino acid transport [GO:0015807]